{
  "term_id": "GO:0006869",
  "term_label": "lipid transport",
  "gene_name": "Sphingosine-1-phosphate transporter SPNS2",
  "gene": "UniProtKB:Q8IVW8",
  "gene_symbol": "SPNS2"
}